{
  "gene": "UniProtKB:Q86YF9",
  "term_label": "BBSome binding",
  "term_id": "GO:0062063",
  "gene_name": "Cilium assembly protein DZIP1",
  "gene_symbol": "DZIP1"
}